{
  "gene_name": "Putative uncharacterized protein COL25A1-DT",
  "gene_symbol": "COL25A1-DT",
  "term_id": "UNKNOWN:0001",
  "term_label": "Unknown molecular function",
  "gene": "UniProtKB:Q6ZST2"
}